Ste12p-Dig1p-Dig2p complex [GO:1990526] (cellular component) References: PMID:16782869 Sources: GOC:rb Definition: A multiprotein complex that is involved in the transcription regulation of mating genes in the yeast S. cerevisiae. Relationships: is_a protein-containing complex [GO:0032991]